{
  "gene_name": "Signal recognition particle 14 kDa protein",
  "gene_symbol": "SRP14",
  "gene": "UniProtKB:P37108",
  "term_id": "GO:0045047",
  "term_label": "protein targeting to ER"
}